{
  "gene": "UniProtKB:P59190",
  "gene_symbol": "RAB15",
  "term_id": "UNKNOWN:0001",
  "term_label": "Unknown molecular function",
  "gene_name": "Ras-related protein Rab-15"
}